{
  "gene_name": "Putative NOL1_NOP2_Sun domain family member 5B",
  "term_label": "Unknown biological process",
  "term_id": "UNKNOWN:0002",
  "gene": "UniProtKB:Q3KNT7",
  "gene_symbol": "NSUN5P1"
}